response to lapatinib [GO:0036274] (biological process) Sources: GOC:hp Note: Note that this term is in the subset of terms that should not be used for direct manual annotation of gene products. It was created to be used for cross-referencing by other ontologies. Direct annotations to this term may be amended during annotation QC. Definition: Any process that results in a change in state or activity of a cell or an organism (in terms of movement, secretion, enzyme production, gene expression, etc.) as a result of a lapatinib stimulus. Relationships: is a type of response to nitrogen compound [GO:1901698]; is a type of GO:1901700